{
  "term_label": "Unknown cellular component",
  "gene_name": "Innate immunity activator protein",
  "term_id": "UNKNOWN:0003",
  "gene": "UniProtKB:Q3KP66",
  "gene_symbol": "INAVA"
}